regulation of RNA metabolic process [GO:0051252] (biological process) Subtypes: regulation of mitochondrial RNA catabolic process [GO:0000960], regulation of RNA stability [GO:0043487], GO:0051253, GO:0051254, GO:0060700, GO:1902374, regulation of mRNA metabolic process [GO:1903311], regulation of snoRNA metabolic process [GO:1903323], regulation of tRNA metabolic process [GO:1903326], GO:1905356, regulation of rRNA processing [GO:2000232], GO:2000628, GO:2001141 Also known as: regulation of RNA metabolism Relationships: is a type of regulation of nucleobase-containing compound metabolic process [GO:0019219]; is a type of GO:0060255; regulates RNA metabolic process [GO:0016070] Definition: Any process that modulates the frequency, rate or extent of the chemical reactions and pathways involving RNA. Sources: GOC:ai